molybdopterin synthase complex [GO:1990140] (cellular component) Relationships: is a type of sulfurtransferase complex [GO:1990228] References: PMID:11135669, PMID:16669776 Sources: GOC:bhm Definition: A heterotetrameric protein complex that catalyses sulfur transfer from the sulfur carrier subunit of molybdopterin synthase to precursor Z to synthesize molybdopterin as part of molybdopterin cofactor (Moco) biosynthesis. In E. coli the subunits are MoaE and MoaD; in human, MOCS2B and MOCS2A. Moco biosynthesis and its constituent molecules are evolutionarily conserved. Also known as: MPT synthase complex, molybdopterin converting factor complex, molybdopterin cofactor (Moco) biosynthesis sulfurtransferase complex